{
  "gene_symbol": "ANKRD1",
  "term_id": "GO:0005634",
  "term_label": "nucleus",
  "gene_name": "Ankyrin repeat domain-containing protein 1",
  "gene": "UniProtKB:Q15327"
}